{
  "gene_symbol": "KCNA10",
  "gene_name": "Potassium voltage-gated channel subfamily A member 10",
  "gene": "UniProtKB:Q16322",
  "term_id": "GO:0016020",
  "term_label": "membrane"
}